{
  "gene_symbol": "IMPG1",
  "term_id": "UNKNOWN:0003",
  "gene": "UniProtKB:Q17R60",
  "gene_name": "Interphotoreceptor matrix proteoglycan 1",
  "term_label": "Unknown cellular component"
}